{
  "term_id": "GO:0004869",
  "gene_name": "Securin-2",
  "term_label": "cysteine-type endopeptidase inhibitor activity",
  "gene": "UniProtKB:Q9NZH5",
  "gene_symbol": "PTTG2"
}